nuclear-transcribed mRNA catabolic process, non-stop decay [GO:0070481] (biological process) Relationships: is a type of nuclear-transcribed mRNA catabolic process [GO:0000956] References: PMID:11910110 Also known as: non-stop decay, non-stop mRNA decay, nonstop mRNA decay, nuclear-transcribed mRNA breakdown, non-stop decay, nuclear-transcribed mRNA catabolism, non-stop decay, nuclear-transcribed mRNA degradation, non-stop decay Definition: The chemical reactions and pathways resulting in the breakdown of the transcript body of a nuclear-transcribed mRNA that is lacking a stop codon.